{
  "gene": "UniProtKB:Q9UKR5",
  "gene_symbol": "ERG28",
  "term_id": "GO:0005783",
  "gene_name": "Ergosterol biosynthetic protein 28 homolog",
  "term_label": "endoplasmic reticulum"
}